{
  "term_id": "GO:0005886",
  "term_label": "plasma membrane",
  "gene_symbol": "LOC124905359",
  "gene_name": "Olfactory receptor",
  "gene": "UniProtKB:A0A0G2JNH3"
}